{
  "gene_symbol": "NTHL1",
  "gene_name": "Endonuclease III-like protein 1",
  "gene": "UniProtKB:P78549",
  "term_label": "nucleus",
  "term_id": "GO:0005634"
}